{
  "gene": "UniProtKB:Q76B58",
  "term_label": "negative regulation of mitotic cell cycle",
  "term_id": "GO:0045930",
  "gene_symbol": "BRINP3",
  "gene_name": "BMP_retinoic acid-inducible neural-specific protein 3"
}